{
  "gene": "UniProtKB:A0A1B0GWH4",
  "gene_symbol": "HSFX3",
  "term_id": "GO:0005634",
  "gene_name": "Heat shock transcription factor, X-linked member 3",
  "term_label": "nucleus"
}